{
  "gene_symbol": "PLA2G5",
  "gene_name": "Phospholipase A2 group V",
  "term_id": "GO:0005509",
  "gene": "UniProtKB:P39877",
  "term_label": "calcium ion binding"
}